{
  "gene_symbol": "AKR1C4",
  "term_label": "progesterone metabolic process",
  "gene": "UniProtKB:P17516",
  "gene_name": "Aldo-keto reductase family 1 member C4",
  "term_id": "GO:0042448"
}